{
  "gene": "UniProtKB:O95343",
  "term_id": "GO:0007420",
  "gene_name": "Homeobox protein SIX3",
  "term_label": "brain development",
  "gene_symbol": "SIX3"
}